{
  "term_label": "Unknown molecular function",
  "term_id": "UNKNOWN:0001",
  "gene": "UniProtKB:Q8TDW7",
  "gene_symbol": "FAT3",
  "gene_name": "Protocadherin Fat 3"
}